propioin synthase activity [GO:0050217] (molecular function) Definition: Catalysis of the reaction: 4-hydroxyhexan-3-one = 2 propanal. Also known as: 4-hydroxy-3-hexanone aldolase activity, 4-hydroxy-3-hexanone propanal-lyase (propanal-forming), 4-hydroxy-3-hexanone propanal-lyase activity Relationships: is a type of GO:0016832 Sources: EC:4.1.2.35, RHEA:11100